{
  "gene_symbol": "FAS",
  "gene_name": "Tumor necrosis factor receptor superfamily member 6",
  "gene": "UniProtKB:P25445",
  "term_id": "GO:0043066",
  "term_label": "negative regulation of apoptotic process"
}